{
  "term_label": "Unknown molecular function",
  "gene": "UniProtKB:Q7L1I2",
  "term_id": "UNKNOWN:0001",
  "gene_name": "Synaptic vesicle glycoprotein 2B",
  "gene_symbol": "SV2B"
}